{
  "gene_symbol": "OR6C68",
  "gene_name": "Olfactory receptor 6C68",
  "term_label": "olfactory receptor activity",
  "gene": "UniProtKB:A6NDL8",
  "term_id": "GO:0004984"
}